host cell chloroplast [GO:0033652] (cellular component) Subtypes: GO:0033653 Relationships: is a type of host cell plastid [GO:0033651] Definition: A chlorophyll-containing plastid as found within host cells with thylakoids organized into grana and frets, or stroma thylakoids, and embedded in a stroma. The host is defined as the larger of the organisms involved in a symbiotic interaction. Sources: GOC:pamgo_curators